{
  "term_label": "nucleus",
  "gene": "UniProtKB:Q9NQ92",
  "gene_symbol": "COPRS",
  "term_id": "GO:0005634",
  "gene_name": "Coordinator of PRMT5 and differentiation stimulator"
}